{
  "gene": "UniProtKB:Q9H6Q3",
  "gene_name": "Src-like-adapter 2",
  "term_label": "Unknown biological process",
  "gene_symbol": "SLA2",
  "term_id": "UNKNOWN:0002"
}